positive regulation of translation initiation in response to endoplasmic reticulum stress [GO:0036494] (biological process) Definition: Any process that activates, or increases the frequency, rate or extent of translation initiation as a result of endoplasmic reticulum stress. Also known as: positive regulation of translation initiation in response to ER stress Relationships: is a type of positive regulation of translational initiation in response to stress [GO:0032058]; is a type of regulation of translation initiation in response to endoplasmic reticulum stress [GO:0036491]; is a type of positive regulation of translation in response to endoplasmic reticulum stress [GO:0036493] Sources: GOC:PARL, GOC:bf